{
  "gene_name": "Tumor protein D52",
  "gene": "UniProtKB:P55327",
  "term_id": "GO:0008284",
  "gene_symbol": "TPD52",
  "term_label": "positive regulation of cell population proliferation"
}